D-ornithine 4,5-aminomutase activity [GO:0047831] (molecular function) Sources: RHEA:14893 Relationships: is_a intramolecular aminotransferase activity [GO:0016869] Also known as: D-alpha-ornithine 5,4-aminomutase activity, D-ornithine aminomutase activity Definition: Catalysis of the reaction: D-ornithine = (2R,4S)-2,4-diaminopentanoate.